N-acetylgalactosamine-6-phosphate deacetylase activity [GO:0047419] (molecular function) Relationships: is a type of hydrolase activity, acting on carbon-nitrogen (but not peptide) bonds, in linear amides [GO:0016811]; is a type of GO:0019213 Definition: Catalysis of the reaction: H2O + N-acetyl-D-galactosamine 6-phosphate = acetate + D-galactosamine 6-phosphate. Sources: RHEA:18149